{
  "gene_name": "Sterol regulatory element-binding protein cleavage-activating protein",
  "term_id": "GO:0045540",
  "term_label": "regulation of cholesterol biosynthetic process",
  "gene": "UniProtKB:Q12770",
  "gene_symbol": "SCAP"
}